lysophospholipid:sodium symporter activity [GO:0051978] (molecular function) Also known as: lysophospholipid transporter activity Sources: GOC:ai Definition: Enables the directed movement of lysophospholipids from one side of a membrane to the other. A lysophospholipid is a phospholipid that lacks one of its fatty acyl chains; it is an intermediate formed during digestion of dietary and biliary phospholipids. Relationships: is a type of phospholipid transporter activity [GO:0005548]; is a type of solute:sodium symporter activity [GO:0015370]; is a type of GO:0015605; is a type of lipid transmembrane transporter activity [GO:0170055]; is a type of GO:1901505; is part of lysophospholipid transport [GO:0051977]